calcium-activated potassium channel activity [GO:0015269] (molecular function) Subtypes: small conductance calcium-activated potassium channel activity [GO:0016286], GO:0022894, large conductance calcium-activated potassium channel activity [GO:0060072] Definition: Enables the transmembrane transfer of a potassium cation by a channel that opens when a calcium cation has been bound by the channel complex or one of its constituent parts. Sources: GOC:dph, GOC:mtg_transport Relationships: is_a GO:0005227; is a type of GO:0005267